{
  "term_id": "GO:0060271",
  "gene": "UniProtKB:O60729",
  "term_label": "cilium assembly",
  "gene_symbol": "CDC14B",
  "gene_name": "Dual specificity protein phosphatase CDC14B"
}